{
  "term_label": "Cul4A-RING E3 ubiquitin ligase complex",
  "gene_symbol": "CRBN",
  "gene": "UniProtKB:Q96SW2",
  "gene_name": "Protein cereblon",
  "term_id": "GO:0031464"
}